{
  "term_label": "Unknown molecular function",
  "gene_name": "RUN domain-containing protein 3A",
  "gene_symbol": "RUNDC3A",
  "term_id": "UNKNOWN:0001",
  "gene": "UniProtKB:Q59EK9"
}